{
  "gene": "UniProtKB:Q9Y5B9",
  "term_label": "nucleosome binding",
  "gene_symbol": "SUPT16H",
  "term_id": "GO:0031491",
  "gene_name": "FACT complex subunit SPT16"
}